regulation of N-terminal peptidyl-lysine acetylation [GO:2000759] (biological process) Definition: Any process that modulates the frequency, rate or extent of N-terminal peptidyl-lysine acetylation. Sources: GOC:obol Relationships: is a type of GO:1903317; is_a regulation of peptidyl-lysine acetylation [GO:2000756]; regulates N-terminal peptidyl-lysine acetylation [GO:0018076] Subtypes: negative regulation of N-terminal peptidyl-lysine acetylation [GO:2000760], GO:2000761